{
  "term_label": "regulation of actin filament length",
  "term_id": "GO:0030832",
  "gene_name": "Myosin-IIIb",
  "gene_symbol": "MYO3B",
  "gene": "UniProtKB:Q8WXR4"
}